{
  "gene_symbol": "DOK2",
  "gene": "UniProtKB:O60496",
  "gene_name": "Docking protein 2",
  "term_label": "transmembrane receptor protein tyrosine kinase adaptor activity",
  "term_id": "GO:0005068"
}